phylloquinone monooxygenase (2,3-epoxidizing) activity [GO:0047097] (molecular function) Sources: RHEA:16745 Definition: Catalysis of the reaction: AH2 + O2 + phylloquinone = 2,3-epoxyphylloquinone + A + H2O. Also known as: phylloquinone epoxidase activity, phylloquinone,hydrogen-donor:oxygen oxidoreductase (2,3-epoxidizing), vitamin K 2,3-epoxidase activity, vitamin K epoxidase activity, vitamin K1 epoxidase activity Relationships: is_a monooxygenase activity [GO:0004497]; is a type of oxidoreductase activity, acting on paired donors, with incorporation or reduction of molecular oxygen [GO:0016705]